{
  "gene_symbol": "MPHOSPH8",
  "gene_name": "M-phase phosphoprotein 8",
  "gene": "UniProtKB:Q99549",
  "term_id": "GO:0005634",
  "term_label": "nucleus"
}